{
  "gene_name": "SUZ domain-containing protein 1",
  "gene": "UniProtKB:Q7Z422",
  "gene_symbol": "SZRD1",
  "term_label": "Unknown biological process",
  "term_id": "UNKNOWN:0002"
}